{
  "gene_name": "Mitochondrial import inner membrane translocase subunit Tim8 A",
  "term_label": "Unknown cellular component",
  "gene": "UniProtKB:O60220",
  "term_id": "UNKNOWN:0003",
  "gene_symbol": "TIMM8A"
}